linoleic acid binding [GO:0070539] (molecular function) Relationships: is a type of GO:0036041 Definition: Binding to linoleic acid, the 18-carbon unsaturated fatty acid (9Z,12Z)-octadeca-9,12-dienoic acid. Sources: GOC:lp, GOC:mah